{
  "term_label": "extracellular space",
  "gene_symbol": "HAMP",
  "gene": "UniProtKB:P81172",
  "term_id": "GO:0005615",
  "gene_name": "Hepcidin"
}